actin filament bundle organization [GO:0061572] (biological process) Sources: GOC:dph Subtypes: actin filament bundle assembly [GO:0051017], actin filament bundle distribution [GO:0070650], formin-nucleated actin cable organization [GO:0110009] Also known as: actin filament cable organization Definition: A process that results in the assembly, arrangement of constituent parts, or disassembly of an actin filament bundle. Relationships: is a type of actin filament organization [GO:0007015]